{
  "gene_name": "Arf-GAP with coiled-coil, ANK repeat and PH domain-containing protein 2",
  "term_id": "GO:0010008",
  "term_label": "endosome membrane",
  "gene_symbol": "ACAP2",
  "gene": "UniProtKB:Q15057"
}